{
  "term_id": "UNKNOWN:0003",
  "gene_name": "Dehydrogenase_reductase SDR family member 9",
  "gene_symbol": "DHRS9",
  "gene": "UniProtKB:Q9BPW9",
  "term_label": "Unknown cellular component"
}